cysteinyl leukotriene receptor activity [GO:0001631] (molecular function) Relationships: is a type of GO:0004974 Definition: Combining with a cysteinyl leukotriene to initiate a change in cell activity. Cysteinyl leukotrienes are leukotrienes that contain a peptide group based on cysteine. Also known as: CysLT receptor Sources: GOC:ai, ISBN:0198506732